{
  "term_label": "Unknown molecular function",
  "gene_symbol": "WDR93",
  "gene_name": "WD repeat-containing protein 93",
  "term_id": "UNKNOWN:0001",
  "gene": "UniProtKB:Q6P2C0"
}